{
  "gene_symbol": "SCIN",
  "gene_name": "Scinderin",
  "term_label": "actin filament binding",
  "gene": "UniProtKB:Q9Y6U3",
  "term_id": "GO:0051015"
}